{
  "gene": "UniProtKB:Q92889",
  "gene_symbol": "ERCC4",
  "term_label": "single-stranded DNA binding",
  "term_id": "GO:0003697",
  "gene_name": "DNA repair endonuclease XPF"
}